kidney smooth muscle cell differentiation [GO:0072195] (biological process) Regulation: regulated by GO:2000356; negatively regulated by negative regulation of kidney smooth muscle cell differentiation [GO:2000357]; positively regulated by positive regulation of kidney smooth muscle cell differentiation [GO:2000358] Sources: GOC:mtg_kidney_jan10 Definition: The process in which a relatively unspecialized cell acquires specialized features of a smooth muscle cell in the kidney. Relationships: is a type of smooth muscle cell differentiation [GO:0051145]; is a type of cell differentiation involved in kidney development [GO:0061005]; is part of kidney smooth muscle tissue development [GO:0072194]